{
  "term_id": "UNKNOWN:0001",
  "term_label": "Unknown molecular function",
  "gene_name": "Thrombospondin type-1 domain-containing protein 7B",
  "gene": "UniProtKB:Q9C0I4",
  "gene_symbol": "THSD7B"
}